{
  "gene_name": "Aldo-keto reductase family 1 member C3",
  "gene_symbol": "AKR1C3",
  "gene": "UniProtKB:P42330",
  "term_id": "GO:0005829",
  "term_label": "cytosol"
}